[protein-PII] uridylyltransferase activity [GO:0008773] (molecular function) Relationships: is a type of uridylyltransferase activity [GO:0070569]; is a type of GO:0140096 Sources: EC:2.7.7.59 Definition: Catalysis of the reaction: UTP + (protein-PII) = diphosphate + uridylyl-(protein-PII). Also known as: uridylyl removing enzyme activity, UTP:[protein-PII] uridylyltransferase activity, PII uridylyl-transferase activity, UTP:protein-PII uridylyltransferase activity, protein-PII uridylyltransferase activity, uridyl removing enzyme